{
  "term_id": "GO:0008201",
  "term_label": "heparin binding",
  "gene": "UniProtKB:O94813",
  "gene_symbol": "SLIT2",
  "gene_name": "Slit homolog 2 protein"
}